{
  "term_label": "protein phosphatase type 1 complex",
  "gene_name": "Protein phosphatase 1 regulatory subunit 3B",
  "term_id": "GO:0000164",
  "gene": "UniProtKB:Q86XI6",
  "gene_symbol": "PPP1R3B"
}